{
  "term_label": "protein folding in endoplasmic reticulum",
  "gene_name": "DnaJ homolog subfamily C member 3",
  "term_id": "GO:0034975",
  "gene": "UniProtKB:Q13217",
  "gene_symbol": "DNAJC3"
}